very-long-chain fatty acyl-CoA dehydrogenase activity [GO:0017099] (molecular function) Note: While there is not universal consensus on the lengths of short-, medium-, long- and very-long-chain fatty acids, the GO uses the definitions in ChEBI (see CHEBI:26666, CHEBI:59554, CHEBI:15904 and CHEBI:27283). Also known as: very long-chain-acyl-CoA dehydrogenase activity, very-long-chain acyl-CoA dehydrogenase activity Definition: Catalysis of the reaction: a very-long-chain 2,3-saturated fatty acyl-CoA + H+ + oxidized [electron-transfer flavoprotein] = a very-long-chain (2E)-enoyl-CoA + reduced [electron-transfer flavoprotein]. A very long-chain fatty acid has an aliphatic tail containing more than 22 carbons. Relationships: is a type of acyl-CoA dehydrogenase activity [GO:0003995] Sources: RHEA:19181